regulation of amylopectin catabolic process [GO:2000945] (biological process) Definition: Any process that modulates the frequency, rate or extent of amylopectin catabolic process. Sources: GOC:mengo_curators Also known as: regulation of Amylopectin catabolism Relationships: is a type of GO:0009894; is_a GO:0060255; regulates amylopectin catabolic process [GO:2000897] Subtypes: GO:2000946, GO:2000947